Cvt vesicle [GO:0033107] (cellular component) References: PMID:15138258 Sources: GOC:rb Definition: A cytosolic vesicle that is enclosed by a double membrane and is implicated in the cytoplasm to vacuole targeting pathway. These vesicles are found in the yeast S. cerevisiae, and contain vacuolar hydrolases, aminopeptidase I (Ape1p) and alpha-mannosidase (Ams1p). Relationships: is a type of GO:0031410 Also known as: cytoplasm to vacuole targeting vesicle, cytoplasm-to-vacuole targeting vesicle